O-phosphoserine sulfhydrylase activity [GO:0033847] (molecular function) Sources: EC:2.5.1.65 Also known as: O-phospho-L-serine:hydrogen-sulfide 2-amino-2-carboxyethyltransferase activity, O-phosphoserine(thiol)-lyase activity Definition: Catalysis of the reaction: O-phospho-L-serine + hydrogen sulfide = L-cysteine + phosphate. Relationships: is a type of GO:0016765